steroid sulfotransferase activity [GO:0050294] (molecular function) Relationships: is a type of sulfotransferase activity [GO:0008146] Also known as: steroid alcohol sulfotransferase, steroid sulphotransferase activity, 3'-phosphoadenylyl-sulfate:phenolic-steroid sulfotransferase activity Definition: Catalysis of the reaction: 3'-phosphoadenosine 5'-phosphosulfate + a phenolic steroid = adenosine 3',5'-bisphosphate + steroid O-sulfate. Sources: MetaCyc:STEROID-SULFOTRANSFERASE-RXN, RHEA:68460